single-stranded telomeric DNA binding [GO:0043047] (molecular function) Sources: GOC:jl, ISBN:0321000382 Also known as: telomeric ssDNA binding Relationships: is a type of GO:0042162; is a type of sequence-specific single stranded DNA binding [GO:0098847] Definition: Binding to single-stranded telomere-associated DNA. Subtypes: C-rich strand telomeric DNA binding [GO:0061730], G-rich strand telomeric DNA binding [GO:0098505]